{
  "gene_name": "DnaJ homolog subfamily C member 12",
  "term_label": "Unknown biological process",
  "gene_symbol": "DNAJC12",
  "gene": "UniProtKB:Q9UKB3",
  "term_id": "UNKNOWN:0002"
}